{
  "term_label": "Unknown molecular function",
  "gene_symbol": "MED9",
  "term_id": "UNKNOWN:0001",
  "gene": "UniProtKB:Q9NWA0",
  "gene_name": "Mediator of RNA polymerase II transcription subunit 9"
}